plus-end-directed vesicle transport along microtubule [GO:0072383] (biological process) Subtypes: plus-end-directed endosome transport along mitotic spindle midzone microtubule [GO:0140024] Definition: The directed movement of a vesicle towards the plus end of a microtubule, mediated by motor proteins. This process begins with the attachment of a vesicle to a microtubule, and ends when the vesicle reaches its final destination. Relationships: is a type of GO:0047496; is a type of plus-end-directed organelle transport along microtubule [GO:0072386] Sources: GOC:BHF, GOC:mah Also known as: microtubule plus-end-directed vesicle localization, microtubule plus-end-directed vesicle distribution